{
  "gene_symbol": "STK11",
  "term_id": "GO:1901610",
  "term_label": "positive regulation of vesicle transport along microtubule",
  "gene_name": "Serine_threonine-protein kinase STK11",
  "gene": "UniProtKB:Q15831"
}